negative regulation of olefin biosynthetic process [GO:1900912] (biological process) Relationships: is a type of negative regulation of biosynthetic process [GO:0009890]; is_a regulation of olefin biosynthetic process [GO:1900911]; negatively regulates olefin biosynthetic process [GO:1900674] Subtypes: negative regulation of ethylene biosynthetic process [GO:0010366], negative regulation of octadecene biosynthetic process [GO:1900915], negative regulation of nonadec-1-ene biosynthetic process [GO:1900936], negative regulation of (Z)-nonadeca-1,14-diene biosynthetic process [GO:1900942], GO:1900948, negative regulation of 18-methylnonadec-1-ene biosynthetic process [GO:1900951], negative regulation of 17-methylnonadec-1-ene biosynthetic process [GO:1900957] Also known as: down regulation of olefin biosynthetic process, down-regulation of olefin biosynthetic process, downregulation of olefin biosynthetic process, inhibition of olefin anabolism, inhibition of olefin biosynthesis, inhibition of olefin biosynthetic process, inhibition of olefin formation, inhibition of olefin synthesis, down regulation of olefin anabolism, down regulation of olefin biosynthesis, down regulation of olefin formation, down regulation of olefin synthesis, down-regulation of olefin anabolism, down-regulation of olefin biosynthesis, down-regulation of olefin formation, down-regulation of olefin synthesis, downregulation of olefin anabolism, downregulation of olefin biosynthesis, downregulation of olefin formation, downregulation of olefin synthesis, negative regulation of olefin anabolism, negative regulation of olefin biosynthesis, negative regulation of olefin formation, negative regulation of olefin synthesis Sources: GOC:TermGenie, GOC:mengo_curators Definition: Any process that stops, prevents or reduces the frequency, rate or extent of olefin biosynthetic process.